{
  "gene": "UniProtKB:Q16665",
  "term_label": "regulation of transcription by RNA polymerase II",
  "term_id": "GO:0006357",
  "gene_symbol": "HIF1A",
  "gene_name": "Hypoxia-inducible factor 1-alpha"
}